positive regulation of monocyte differentiation [GO:0045657] (biological process) Definition: Any process that activates or increases the frequency, rate or extent of monocyte differentiation. Sources: GOC:go_curators Also known as: up regulation of monocyte differentiation, up-regulation of monocyte differentiation, upregulation of monocyte differentiation, activation of monocyte differentiation, stimulation of monocyte differentiation Relationships: is a type of GO:0002763; is a type of GO:0045655; positively regulates monocyte differentiation [GO:0030224]